maternal specification of dorsal/ventral axis, oocyte, soma encoded [GO:0007313] (biological process) Sources: GOC:dph, GOC:mtg_sensu, GOC:tb, ISBN:0879694238 Definition: Polarization of the oocyte along the dorsal-ventral axis, by a gene product encoded by somatic cells. An example of this is found in Drosophila melanogaster. Relationships: is a type of oocyte dorsal/ventral axis specification [GO:0007310] Also known as: maternal determination of dorsal/ventral axis, oocyte, soma encoded, maternal specification of dorsal-ventral axis, oocyte, soma encoded, maternal specification of dorsoventral axis, oocyte, soma encoded